{
  "gene": "UniProtKB:O75616",
  "term_label": "rRNA binding",
  "gene_name": "GTPase Era, mitochondrial",
  "term_id": "GO:0019843",
  "gene_symbol": "ERAL1"
}